{
  "gene_name": "Zinc finger matrin-type protein 4",
  "term_id": "UNKNOWN:0002",
  "term_label": "Unknown biological process",
  "gene": "UniProtKB:Q9H898",
  "gene_symbol": "ZMAT4"
}